{
  "gene_name": "Nuclear pore complex protein Nup153",
  "term_id": "GO:0006606",
  "term_label": "protein import into nucleus",
  "gene": "UniProtKB:P49790",
  "gene_symbol": "NUP153"
}